{
  "term_id": "GO:0009154",
  "gene_name": "Adenosine 5'-monophosphoramidase HINT1",
  "gene": "UniProtKB:P49773",
  "term_label": "purine ribonucleotide catabolic process",
  "gene_symbol": "HINT1"
}